alginate synthase activity [GO:0047643] (molecular function) Definition: Catalysis of the reaction: GDP-D-mannuronate + alginate(n) = GDP + alginate(n+1). Sources: EC:2.4.1.33, MetaCyc:ALGINATE-SYNTHASE-RXN Relationships: is a type of GO:0016758 Also known as: GDP-D-mannuronate:alginate D-mannuronyltransferase activity, mannuronosyl transferase activity